metanephric glomerular parietal epithelial cell differentiation [GO:0072245] (biological process) Sources: GOC:mtg_kidney_jan10 Definition: The process in which a relatively unspecialized cell acquires specialized features of a metanephric glomerular parietal epithelial cell. Metanephric glomerular parietal epithelial cells are specialized epithelial cells that form tight junctions as a barrier to protein transport. Relationships: is a type of glomerular parietal epithelial cell differentiation [GO:0072139]; is a type of metanephric glomerular epithelial cell differentiation [GO:0072312]